{
  "term_id": "GO:0016567",
  "gene": "UniProtKB:O00237",
  "term_label": "protein ubiquitination",
  "gene_name": "E3 ubiquitin-protein ligase RNF103",
  "gene_symbol": "RNF103"
}